semicircular canal fusion [GO:0060879] (biological process) Definition: Creation of the central hole of the semicircular canal by sealing the edges of the pouch that forms during the process of semicircular canal formation. Relationships: is_a GO:0060606; is part of semicircular canal formation [GO:0060876] Sources: GOC:dph, GOC:sdb_2009, GOC:tb